adenosine kinase activity [GO:0004001] (molecular function) Relationships: is a type of nucleoside kinase activity [GO:0019206]; is part of AMP biosynthetic process [GO:0006167] References: PMID:11223943 Sources: EC:2.7.1.20 Also known as: adenosine 5-phosphotransferase activity, ATP:adenosine 5'-phosphotransferase activity, adenosine kinase (phosphorylating) Definition: Catalysis of the reaction: ATP + adenosine = ADP + AMP.